lactate biosynthetic process [GO:0019249] (biological process) Relationships: is_a GO:0006089; is a type of GO:0072330 Subtypes: lactate biosynthetic process from pyruvate [GO:0019244], D-lactate biosynthetic process from methylglyoxal via (R)-lactaldehyde [GO:0019248], GO:0036530 Sources: GOC:go_curators Definition: The chemical reactions and pathways resulting in the formation of lactate, the anion of lactic acid. Also known as: lactate anabolism, lactate biosynthesis, lactate formation, lactate synthesis